{
  "gene": "UniProtKB:Q86WS3",
  "gene_symbol": "OOSP2",
  "term_id": "UNKNOWN:0002",
  "gene_name": "Oocyte-secreted protein 2",
  "term_label": "Unknown biological process"
}